{
  "gene_name": "Flap endonuclease 1",
  "gene_symbol": "FEN1",
  "term_label": "magnesium ion binding",
  "term_id": "GO:0000287",
  "gene": "UniProtKB:P39748"
}